{
  "term_id": "GO:0004984",
  "gene_name": "Olfactory receptor 5H14",
  "term_label": "olfactory receptor activity",
  "gene_symbol": "OR5H14",
  "gene": "UniProtKB:A6NHG9"
}